{
  "term_id": "GO:0097526",
  "gene_symbol": "SNRPG",
  "term_label": "spliceosomal tri-snRNP complex",
  "gene_name": "Small nuclear ribonucleoprotein G",
  "gene": "UniProtKB:P62308"
}